{
  "gene_name": "Zinc finger protein 738",
  "term_id": "GO:0003700",
  "gene": "UniProtKB:Q8NE65",
  "gene_symbol": "ZNF738",
  "term_label": "DNA-binding transcription factor activity"
}